{
  "term_label": "mRNA export from nucleus",
  "gene_name": "THO complex subunit 1",
  "term_id": "GO:0006406",
  "gene_symbol": "THOC1",
  "gene": "UniProtKB:Q96FV9"
}